plus-end specific microtubule depolymerization [GO:0070462] (biological process) Relationships: is a type of microtubule depolymerization [GO:0007019] Definition: The removal of tubulin heterodimers from the plus end of a microtubule. References: PMID:16906145, PMID:16906148 Sources: GOC:krc